{
  "term_id": "GO:0015179",
  "gene_name": "Putative sodium-coupled neutral amino acid transporter 8",
  "gene": "UniProtKB:A6NNN8",
  "term_label": "L-amino acid transmembrane transporter activity",
  "gene_symbol": "SLC38A8"
}